{
  "gene_name": "Neuroblastoma breakpoint family member 26",
  "gene": "UniProtKB:B4DH59",
  "term_id": "UNKNOWN:0003",
  "gene_symbol": "NBPF26",
  "term_label": "Unknown cellular component"
}